{
  "gene_symbol": "BRSK1",
  "term_label": "establishment of cell polarity",
  "gene_name": "Serine_threonine-protein kinase BRSK1",
  "term_id": "GO:0030010",
  "gene": "UniProtKB:Q8TDC3"
}